troponin C binding [GO:0030172] (MF) Relationships: is a type of cytoskeletal protein binding [GO:0008092] Definition: Binding to troponin C, the calcium-binding subunit of the troponin complex. Sources: GOC:mah, ISBN:0815316194